{
  "gene_name": "Antileukoproteinase",
  "gene_symbol": "SLPI",
  "gene": "UniProtKB:P03973",
  "term_label": "serine-type endopeptidase inhibitor activity",
  "term_id": "GO:0004867"
}